{
  "term_id": "GO:0000902",
  "term_label": "cell morphogenesis",
  "gene_symbol": "CDH8",
  "gene": "UniProtKB:P55286",
  "gene_name": "Cadherin-8"
}